{
  "term_id": "UNKNOWN:0003",
  "gene": "UniProtKB:O95455",
  "term_label": "Unknown cellular component",
  "gene_name": "dTDP-D-glucose 4,6-dehydratase",
  "gene_symbol": "TGDS"
}